cGAS/STING signaling pathway [GO:0140896] (biological process) References: PMID:27648547, PMID:34261127, PMID:34261128 Regulation: positively regulated by positive regulation of cGAS/STING signaling pathway [GO:0141111]; negatively regulated by negative regulation of cGAS/STING signaling pathway [GO:0160049] Definition: The series of molecular signals initiated by the binding of a double-stranded DNA or RNA from another organism to cytosolic cyclic GMP-AMP (cGAMP) synthase (cGAS) that activates innate immune responses through production of the second messenger cGAMP, which activates the adaptor STING. Relationships: is a type of GO:0002753